nigerotriose transport [GO:2001091] (biological process) Relationships: is a type of trisaccharide transport [GO:2001088] Regulation: regulated by regulation of nigerotriose transport [GO:1900357]; negatively regulated by GO:1900358; positively regulated by GO:1900359 Sources: GOC:mengo_curators Definition: The directed movement of a nigerotrioseacetate into, out of or within a cell, or between cells, by means of some agent such as a transporter or pore.